{
  "term_label": "release of sequestered calcium ion into cytosol",
  "gene": "UniProtKB:O75038",
  "gene_name": "1-phosphatidylinositol 4,5-bisphosphate phosphodiesterase eta-2",
  "gene_symbol": "PLCH2",
  "term_id": "GO:0051209"
}